{
  "gene_name": "DNA-directed RNA polymerase III subunit RPC8",
  "term_label": "Unknown molecular function",
  "term_id": "UNKNOWN:0001",
  "gene_symbol": "POLR3H",
  "gene": "UniProtKB:Q9Y535"
}